{
  "gene_symbol": "NMT2",
  "term_label": "glycylpeptide N-tetradecanoyltransferase activity",
  "gene": "UniProtKB:O60551",
  "term_id": "GO:0004379",
  "gene_name": "Glycylpeptide N-tetradecanoyltransferase 2"
}